{
  "gene_name": "Vesicle-associated membrane protein 2",
  "term_id": "GO:0006906",
  "gene": "UniProtKB:P63027",
  "gene_symbol": "VAMP2",
  "term_label": "vesicle fusion"
}